{
  "gene_symbol": "KCNQ1",
  "gene": "UniProtKB:P51787",
  "term_label": "potassium ion export across plasma membrane",
  "term_id": "GO:0097623",
  "gene_name": "Potassium voltage-gated channel subfamily KQT member 1"
}